{
  "term_label": "cell adhesion molecule binding",
  "gene_symbol": "PCDHGB6",
  "gene": "UniProtKB:Q9Y5F9",
  "term_id": "GO:0050839",
  "gene_name": "Protocadherin gamma-B6"
}